N-acetylgalactosamine 4-sulfate 6-O-sulfotransferase activity [GO:0050659] (molecular function) Also known as: 3'-phosphoadenylyl-sulfate:dermatan 6'-sulfotransferase activity, GalNAc4S-6ST, N-acetylgalactosamine 4-sulfate 6-O-sulphotransferase activity Relationships: is a type of GO:0008146 Sources: EC:2.8.2.33 Definition: Catalysis of the reactions: n 3'-phosphoadenylyl sulfate + chondroitin 4'-sulfate = n adenosine 3',5'-bisphosphate + chondroitin 4',6'-bissulfate + n H+, and n 3'-phosphoadenylyl sulfate + dermatan 4'-sulfate = n adenosine 3',5'-bisphosphate + dermatan 4',6'-bissulfate + n H+.